{
  "gene_symbol": "PCDHB3",
  "term_id": "GO:0050839",
  "term_label": "cell adhesion molecule binding",
  "gene_name": "Protocadherin beta-3",
  "gene": "UniProtKB:Q9Y5E6"
}